{
  "gene": "UniProtKB:Q9UM21",
  "term_label": "protein N-linked glycosylation",
  "gene_symbol": "MGAT4A",
  "gene_name": "Alpha-1,3-mannosyl-glycoprotein 4-beta-N-acetylglucosaminyltransferase A",
  "term_id": "GO:0006487"
}